apical dendrite [GO:0097440] (cellular component) Sources: NIF_Subcellular:sao273773228 Subtypes: GO:0150014, apical proximal dendrite [GO:0150015] Definition: A dendrite that emerges near the apical pole of a neuron. In bipolar neurons, apical dendrites are located on the opposite side of the soma from the axon. Relationships: is a type of GO:0030425